protein demethylation [GO:0006482] (biological process) Definition: The removal of a methyl group, from a protein amino acid. A methyl group is derived from methane by the removal of a hydrogen atom. Also known as: protein amino acid demethylation Subtypes: C-terminal protein demethylation [GO:1990577] Relationships: is a type of protein dealkylation [GO:0008214]; is a type of demethylation [GO:0070988] Sources: GOC:mah